{
  "term_id": "GO:0005615",
  "gene": "UniProtKB:P39905",
  "gene_name": "Glial cell line-derived neurotrophic factor",
  "term_label": "extracellular space",
  "gene_symbol": "GDNF"
}